{
  "term_id": "GO:0000981",
  "gene_name": "Transcription factor 7-like 1",
  "gene": "UniProtKB:Q9HCS4",
  "term_label": "DNA-binding transcription factor activity, RNA polymerase II-specific",
  "gene_symbol": "TCF7L1"
}